regulation of sporangiospore formation [GO:0075286] (biological process) Relationships: is a type of regulation of asexual sporulation resulting in formation of a cellular spore [GO:0043943]; regulates GO:0034300 Sources: GOC:pamgo_curators Definition: Any process that modulates the frequency, rate or extent of sporangiospore formation, a process in which sporangiospores, a type of asexual spore found in fungi, are formed. Sporangiospores are formed within sac-like structure, the sporangium, following the division of the cytoplasm. Subtypes: GO:0075240, positive regulation of sporangiospore formation [GO:0075287], negative regulation of sporangiospore formation [GO:0075288], regulation of aplanospore formation [GO:0075290]